{
  "term_label": "ribonucleoprotein complex",
  "gene_name": "Heterogeneous nuclear ribonucleoprotein H3",
  "gene": "UniProtKB:P31942",
  "term_id": "GO:1990904",
  "gene_symbol": "HNRNPH3"
}